{
  "gene_symbol": "ASCL4",
  "gene": "UniProtKB:Q6XD76",
  "term_label": "RNA polymerase II transcription regulator complex",
  "gene_name": "Achaete-scute homolog 4",
  "term_id": "GO:0090575"
}